{
  "term_label": "Unknown molecular function",
  "gene_symbol": "CCDC54",
  "term_id": "UNKNOWN:0001",
  "gene_name": "Coiled-coil domain-containing protein 54",
  "gene": "UniProtKB:Q8NEL0"
}